{
  "term_label": "positive regulation of monocyte chemotaxis",
  "gene": "UniProtKB:Q9HCY8",
  "term_id": "GO:0090026",
  "gene_name": "Protein S100-A14",
  "gene_symbol": "S100A14"
}